{
  "gene": "UniProtKB:Q96SF2",
  "term_label": "protein folding",
  "gene_name": "T-complex protein 1 subunit theta-like 2",
  "gene_symbol": "CCT8L2",
  "term_id": "GO:0006457"
}